{
  "gene_symbol": "IQCG",
  "term_id": "GO:0005737",
  "term_label": "cytoplasm",
  "gene_name": "Dynein regulatory complex protein 9",
  "gene": "UniProtKB:Q9H095"
}